{
  "term_id": "GO:0000981",
  "gene_symbol": "ZNF701",
  "gene": "UniProtKB:Q9NV72",
  "gene_name": "Zinc finger protein 701",
  "term_label": "DNA-binding transcription factor activity, RNA polymerase II-specific"
}